{
  "term_label": "Unknown molecular function",
  "gene": "UniProtKB:Q9HBJ0",
  "gene_name": "Placenta-specific protein 1",
  "gene_symbol": "PLAC1",
  "term_id": "UNKNOWN:0001"
}